cell communication by electrical coupling involved in cardiac conduction [GO:0086064] (biological process) Definition: The process that mediates signaling interactions between one cell and another cell by transfer of current between their adjacent cytoplasms via intercellular protein channels and contributes to the process of cardiac conduction. Subtypes: SA node cell to atrial cardiac muscle cell communication by electrical coupling [GO:0086021], atrial cardiac muscle cell to AV node cell communication by electrical coupling [GO:0086044], GO:0086053, bundle of His cell to Purkinje myocyte communication by electrical coupling [GO:0086054], Purkinje myocyte to ventricular cardiac muscle cell communication by electrical coupling [GO:0086055] Sources: GOC:BHF, GOC:mtg_cardiac_conduct_nov11 Relationships: is a type of cell communication by electrical coupling [GO:0010644]; is a type of cell communication involved in cardiac conduction [GO:0086065] Regulation: regulated by GO:1901844; negatively regulated by negative regulation of cell communication by electrical coupling involved in cardiac conduction [GO:1901845]; positively regulated by positive regulation of cell communication by electrical coupling involved in cardiac conduction [GO:1901846]